{
  "gene_symbol": "LINC02694",
  "term_id": "UNKNOWN:0003",
  "term_label": "Unknown cellular component",
  "gene": "UniProtKB:Q8NAA6",
  "gene_name": "Putative uncharacterized protein encoded by LINC02694"
}